{
  "term_label": "chromatin",
  "gene": "UniProtKB:Q9ULW6",
  "gene_name": "Nucleosome assembly protein 1-like 2",
  "gene_symbol": "NAP1L2",
  "term_id": "GO:0000785"
}